regulation of exit from meiosis [GO:0106060] (biological process) References: PMID:11493649 Sources: GOC:al Subtypes: negative regulation of exit from meiosis [GO:0106061], positive regulation of exit from meiosis [GO:0106062] Relationships: is a type of regulation of meiotic cell cycle phase transition [GO:1901993]; regulates GO:1990947 Definition: Any process that modulates the frequency, rate or extent of exit from mitosis.